{
  "gene_name": "Olfactory receptor 11H12",
  "term_id": "UNKNOWN:0001",
  "term_label": "Unknown molecular function",
  "gene_symbol": "OR11H12",
  "gene": "UniProtKB:B2RN74"
}